snRNA pseudouridine synthase activity [GO:0106032] (molecular function) Definition: Catalysis of the reaction: uridine in snRNA = pseudouridine in snRNA. Conversion of uridine in an snRNA molecule to pseudouridine by rotation of the C1'-N-1 glycosidic bond of uridine in RNA to a C1'-C5. Relationships: is a type of GO:0009982; is a type of catalytic activity, acting on RNA [GO:0140098] References: PMID:28432181 Sources: RHEA:51124